(S)-canadine synthase activity [GO:0047056] (molecular function) Sources: RHEA:21456 Definition: Catalysis of the reaction: (S)-tetrahydrocolumbamine + reduced [NADPH--hemoprotein reductase] + O2 = (S)-canadine + oxidized [NADPH--hemoprotein reductase] + 2 H2O + H+. Relationships: is_a oxidoreductase activity, acting on paired donors, with oxidation of a pair of donors resulting in the reduction of molecular oxygen to two molecules of water [GO:0016717] Also known as: (S)-tetrahydroberberine synthase activity, (S)-tetrahydrocolumbamine oxidase (methylenedioxy-bridge-forming) activity